midbody abscission [GO:0061952] (BP) References: PMID:12737809, PMID:29903934 Definition: The process by which the midbody, the cytoplasmic bridge that connects the two prospective daughter cells, is severed at the end of mitotic cytokinesis, resulting in two separate daughter cells. Also known as: cell separation during cytokinesis, cytokinetic abscission Relationships: is a type of membrane organization [GO:0061024]; is_a mitotic cytokinetic process [GO:1902410]